{
  "gene_symbol": "PICALM",
  "term_label": "phosphatidylinositol-4,5-bisphosphate binding",
  "gene": "UniProtKB:Q13492",
  "gene_name": "Phosphatidylinositol-binding clathrin assembly protein",
  "term_id": "GO:0005546"
}